{
  "term_id": "GO:0043022",
  "gene_symbol": "MAIP1",
  "gene_name": "m-AAA protease-interacting protein 1, mitochondrial",
  "term_label": "ribosome binding",
  "gene": "UniProtKB:Q8WWC4"
}